microfibril [GO:0001527] (cellular component) Relationships: is a type of supramolecular fiber [GO:0099512]; BFO_0000050 GO:0031012 References: PMID:27026396 Also known as: extended fibrils, fibrillin Definition: Extracellular matrix components occurring independently or along with elastin. Thought to have force-bearing functions in tendon. In addition to fibrillins, microfibrils may contain other associated proteins.